dolichyl pyrophosphate Glc2Man9GlcNAc2 alpha-1,2-glucosyltransferase activity [GO:0106073] (MF) Relationships: is a type of dolichyl-phosphate-glucose-glycolipid alpha-glucosyltransferase activity [GO:0004583] References: PMID:9597543 Sources: GOC:ha Definition: Catalysis of the addition of the third glucose residue to the lipid-linked oligosaccharide precursor for N-linked glycosylation; the transfer of glucose from dolichyl phosphate glucose (Dol-P-Glc) on to the lipid-linked oligosaccharide Glc(2)Man(9)GlcNAc(2)-PP-Dol.